{
  "gene_symbol": "KLB",
  "term_label": "Unknown biological process",
  "gene_name": "Beta-klotho",
  "term_id": "UNKNOWN:0002",
  "gene": "UniProtKB:Q86Z14"
}